{
  "term_id": "GO:0005739",
  "gene": "UniProtKB:Q9BUK0",
  "term_label": "mitochondrion",
  "gene_name": "Coiled-coil-helix-coiled-coil-helix domain-containing protein 7",
  "gene_symbol": "CHCHD7"
}